dihydrolipoamide metabolic process [GO:0051068] (biological process) Definition: The chemical reactions and pathways involving dihydrolipoamide, the reduced form of lipoamide, produced as an intermediate in the reactions in which lipoamide acts as a cofactor. Relationships: is a type of sulfur compound metabolic process [GO:0006790]; is a type of GO:0043603 Also known as: dihydrolipoamide metabolism, dihydrothioctamide metabolic process, dihydrothioctamide metabolism, dihydrolipoamide reduction Sources: ISBN:0721601464